{
  "gene": "UniProtKB:Q9Y6M0",
  "gene_symbol": "PRSS21",
  "term_label": "spermatogenesis",
  "term_id": "GO:0007283",
  "gene_name": "Testisin"
}